A axonemal microtubule [GO:0097649] (cellular component) Also known as: A tubule Definition: A complete microtubule with 13 protofilaments that fuses with an incomplete microtubule called B tubule (containing 10 protofilaments only) to form an axonemal outer doublet. Inner and outer dynein arms, as well as the radial spoke, are attached to the A tubule. Sources: GOC:cilia, ISBN:0716731363 Relationships: is a type of GO:0005879; is part of axonemal doublet microtubule [GO:0097545]